{
  "gene_name": "Adenine DNA glycosylase",
  "gene_symbol": "MUTYH",
  "term_id": "GO:0005634",
  "term_label": "nucleus",
  "gene": "UniProtKB:Q9UIF7"
}